{
  "gene_name": "6-pyruvoyl tetrahydrobiopterin synthase",
  "gene_symbol": "PTS",
  "term_id": "GO:0005739",
  "term_label": "mitochondrion",
  "gene": "UniProtKB:Q03393"
}